{
  "gene_symbol": "CA14",
  "term_id": "GO:0004089",
  "gene_name": "Carbonic anhydrase 14",
  "term_label": "carbonate dehydratase activity",
  "gene": "UniProtKB:Q9ULX7"
}